{
  "term_label": "ubiquitin protein ligase activity",
  "gene": "UniProtKB:Q9H0M0",
  "gene_symbol": "WWP1",
  "gene_name": "NEDD4-like E3 ubiquitin-protein ligase WWP1",
  "term_id": "GO:0061630"
}